N-acetylmuramic acid metabolic process [GO:0097172] (biological process) Sources: GOC:yaf Relationships: is_a GO:0019752 Subtypes: N-acetylmuramic acid catabolic process [GO:0097173] Definition: The chemical reactions and pathways involving N-acetylmuramic acid (MurNAc), a monosaccharide derivative of N-acetylglucosamine. Also known as: N-acetylmuramate metabolic process, N-acetylmuramate metabolism, N-acetylmuramic acid metabolism